{
  "gene_symbol": "GPR32P1",
  "gene": "UniProtKB:Q8NGA4",
  "term_label": "N-formyl peptide receptor activity",
  "term_id": "GO:0004982",
  "gene_name": "Putative G-protein coupled receptor GPR32P1"
}